competence pheromone activity [GO:0030413] (molecular function) Relationships: is a type of GO:0005186 Definition: A small peptide excreted by a naturally transformable bacterium (e.g. Bacillus subtilis) that transmits a signal required for the establishment of competence. References: PMID:7698645 Sources: GOC:mah